{
  "gene_symbol": "OR4N4",
  "gene_name": "Olfactory receptor 4N4",
  "gene": "UniProtKB:Q8N0Y3",
  "term_label": "olfactory receptor activity",
  "term_id": "GO:0004984"
}